post-embryonic medial fin morphogenesis [GO:0035132] (biological process) Definition: The process, occurring after embryonic development, by which the anatomical structures of the medial fin are generated and organized. Medial fins are unpaired fins of fish, usually located dorsomedially or ventromedially and primarily used for stability while swimming. Sources: GOC:dgh Also known as: post-embryonic unpaired fin morphogenesis Relationships: is a type of post-embryonic appendage morphogenesis [GO:0035120]; is a type of medial fin morphogenesis [GO:0035141] Subtypes: post-embryonic caudal fin morphogenesis [GO:0035133], post-embryonic dorsal fin morphogenesis [GO:0035134], GO:0035135